{
  "gene_name": "Interferon-inducible protein AIM2",
  "gene_symbol": "AIM2",
  "term_id": "GO:0002218",
  "term_label": "activation of innate immune response",
  "gene": "UniProtKB:O14862"
}